sperm flagellum [GO:0036126] (cellular component) Definition: A microtubule-based flagellum (or cilium) that is part of a sperm, a mature male germ cell that develops from a spermatid. Note: Note that cilia and eukaryotic flagella are deemed to be equivalent. In this case community usage is always 'flagellum', hence the primary term name, but the cilium parentage is deliberate. Also known as: sperm cilium, sperm tail Relationships: is a type of GO:0097729 References: PMID:8441407 Sources: GOC:cilia, GOC:sart